{
  "gene_symbol": "DBNDD1",
  "term_id": "UNKNOWN:0003",
  "gene": "UniProtKB:Q9H9R9",
  "term_label": "Unknown cellular component",
  "gene_name": "Dysbindin domain-containing protein 1"
}